{
  "term_id": "GO:1901981",
  "gene": "UniProtKB:P17677",
  "gene_symbol": "GAP43",
  "term_label": "phosphatidylinositol phosphate binding",
  "gene_name": "Neuromodulin"
}